{
  "term_id": "GO:0007099",
  "gene": "UniProtKB:O43379",
  "gene_symbol": "WDR62",
  "gene_name": "WD repeat-containing protein 62",
  "term_label": "centriole replication"
}